oncostatin-M receptor binding [GO:0005147] (molecular function) Also known as: oncostatin-M, oncostatin-M receptor ligand Definition: Binding to an oncostatin-M receptor. Sources: GOC:ai Relationships: is a type of cytokine receptor binding [GO:0005126]